{
  "term_label": "G protein-coupled receptor activity",
  "term_id": "GO:0004930",
  "gene_symbol": "GPR35",
  "gene": "UniProtKB:Q9HC97",
  "gene_name": "G-protein coupled receptor 35"
}